thymine transport [GO:0035364] (biological process) Regulation: RO_0002211 by regulation of thymine transport [GO:0035365]; negatively regulated by negative regulation of thymine transport [GO:0035366]; positively regulated by positive regulation of thymine transport [GO:0035367] Relationships: is a type of pyrimidine nucleobase transport [GO:0015855] Also known as: 5-methyluracil transport, thymine transmembrane transport Sources: GO:sl Definition: The directed movement of thymine, 5-methyluracil, into, out of or within a cell, or between cells, by means of some agent such as a transporter or pore.